{
  "term_label": "plasma membrane",
  "gene": "UniProtKB:P20648",
  "gene_symbol": "ATP4A",
  "gene_name": "Potassium-transporting ATPase alpha chain 1",
  "term_id": "GO:0005886"
}